enterobactin biosynthetic process [GO:0009239] (biological process) Sources: GOC:go_curators Also known as: enterobactin anabolism, enterobactin biosynthesis, enterobactin formation, enterobactin synthesis, enterochelin biosynthesis, enterochelin biosynthetic process, enterobactin biosynthetic process, peptide formation, enterobactin biosynthetic process, peptide modification, enterobactin synthetase Relationships: is a type of catechol-containing siderophore biosynthetic process [GO:0019540]; is_a macrolide biosynthetic process [GO:0033068] Definition: The chemical reactions and pathways resulting in the formation of enterobactin, a catechol-derived siderochrome of Enterobacteria; enterobactin (N',N',N''-(2,6,10-trioxo-1,5,9-triacyclodecane-3,7,11-triyl)tris(2,3-dihydroxy)benzamide) is a self-triester of 2,3-dihydroxy-N-benzoyl-L-serine and a product of the shikimate pathway.